metanephric part of ureteric bud development [GO:0035502] (biological process) Sources: GOC:mtg_kidney_jan10 Definition: The development of the portion of the ureteric bud tube that contributes to the morphogenesis of the metanephros. Regulation: regulated by regulation of metanephric ureteric bud development [GO:2001074]; RO_0002212 by negative regulation of metanephric ureteric bud development [GO:2001075]; positively regulated by positive regulation of metanephric ureteric bud development [GO:2001076] Relationships: is a type of tube development [GO:0035295]; is part of ureteric bud development [GO:0001657]; BFO_0000050 metanephros morphogenesis [GO:0003338]